{
  "gene_symbol": "ATP8B2",
  "term_label": "Golgi organization",
  "term_id": "GO:0007030",
  "gene_name": "Phospholipid-transporting ATPase ID",
  "gene": "UniProtKB:P98198"
}